{
  "term_id": "UNKNOWN:0002",
  "gene": "UniProtKB:Q8TE69",
  "gene_symbol": "EOLA1",
  "gene_name": "Protein EOLA1",
  "term_label": "Unknown biological process"
}